{
  "term_id": "GO:0005768",
  "gene": "UniProtKB:Q8IUC6",
  "gene_symbol": "TICAM1",
  "gene_name": "TIR domain-containing adapter molecule 1",
  "term_label": "endosome"
}